{
  "term_id": "GO:0086036",
  "gene": "UniProtKB:Q13061",
  "term_label": "regulation of cardiac muscle cell membrane potential",
  "gene_name": "Triadin",
  "gene_symbol": "TRDN"
}